{
  "gene_symbol": "CT62",
  "term_label": "Unknown cellular component",
  "gene_name": "Cancer_testis antigen 62",
  "gene": "UniProtKB:P0C5K7",
  "term_id": "UNKNOWN:0003"
}